{
  "gene_symbol": "ATP5F1A",
  "gene": "UniProtKB:P25705",
  "term_label": "proton motive force-driven ATP synthesis",
  "term_id": "GO:0015986",
  "gene_name": "ATP synthase subunit alpha, mitochondrial"
}